{
  "gene_symbol": "PRXL2A",
  "gene_name": "Peroxiredoxin-like 2A",
  "gene": "UniProtKB:Q9BRX8",
  "term_label": "Unknown biological process",
  "term_id": "UNKNOWN:0002"
}